{
  "term_id": "UNKNOWN:0002",
  "gene_symbol": "CCDC7",
  "gene": "UniProtKB:Q96M83",
  "term_label": "Unknown biological process",
  "gene_name": "Coiled-coil domain-containing protein 7"
}